{
  "gene": "UniProtKB:Q9UPW5",
  "gene_name": "Cytosolic carboxypeptidase 1",
  "term_id": "GO:0015630",
  "gene_symbol": "AGTPBP1",
  "term_label": "microtubule cytoskeleton"
}